{
  "gene_symbol": "CACNG7",
  "gene": "UniProtKB:P62955",
  "gene_name": "Voltage-dependent calcium channel gamma-7 subunit",
  "term_id": "GO:0032281",
  "term_label": "AMPA glutamate receptor complex"
}